negative regulation of hydrogen peroxide biosynthetic process [GO:0010730] (biological process) Also known as: negative regulation of hydrogen peroxide biosynthesis Sources: GOC:dph, GOC:hjd, GOC:tb Definition: Any process that decreases the rate, frequency or extent of hydrogen peroxide biosynthesis. The chemical reactions and pathways resulting in the formation of hydrogen peroxide (H2O2), a potentially harmful byproduct of aerobic cellular respiration which can cause damage to DNA. Relationships: is a type of negative regulation of hydrogen peroxide metabolic process [GO:0010727]; is a type of GO:0010728; is a type of negative regulation of reactive oxygen species biosynthetic process [GO:1903427]; negatively regulates hydrogen peroxide biosynthetic process [GO:0050665]